{
  "term_label": "neuromuscular junction",
  "term_id": "GO:0031594",
  "gene": "UniProtKB:Q86WN1",
  "gene_name": "F-BAR and double SH3 domains protein 1",
  "gene_symbol": "FCHSD1"
}